{
  "gene_name": "Myosin-10",
  "term_label": "myosin II complex",
  "term_id": "GO:0016460",
  "gene_symbol": "MYH10",
  "gene": "UniProtKB:P35580"
}